MHC class I protein binding [GO:0042288] (molecular function) Relationships: is a type of GO:0042287 Subtypes: MHC class I protein binding, via antigen binding groove [GO:0023027], GO:0023028 Also known as: major histocompatibility complex class I binding, major histocompatibility complex class I ligand, T cell receptor activity, alpha-beta T cell receptor activity, gamma-delta T cell receptor activity Definition: Binding to a major histocompatibility complex class I molecule; a set of molecules displayed on cell surfaces that are responsible for lymphocyte recognition and antigen presentation. Note: Note that this term does not include binding to the antigen peptide bound to the MHC protein. Consider also annotating to the molecular function term 'peptide antigen binding ; GO:0042605' or one of its children. Sources: GOC:jl